{
  "term_label": "Unknown biological process",
  "gene_name": "Coiled-coil domain-containing protein 153",
  "gene_symbol": "CCDC153",
  "term_id": "UNKNOWN:0002",
  "gene": "UniProtKB:Q494R4"
}